regulation of hemocyte proliferation [GO:0035206] (biological process) Relationships: is a type of GO:0002682; is a type of regulation of cell population proliferation [GO:0042127]; is a type of GO:0050793; is a type of regulation of multicellular organismal process [GO:0051239]; regulates hemocyte proliferation [GO:0035172] Sources: GOC:bf, GOC:mtg_sensu Also known as: regulation of arthropod blood cell proliferation Definition: Any process that modulates the frequency, rate or extent of hemocyte proliferation. Hemocytes are blood cells associated with a hemocoel (the cavity containing most of the major organs of the arthropod body) which are involved in defense and clotting of hemolymph, but not involved in transport of oxygen. An example of this is found in Drosophila melanogaster. Subtypes: negative regulation of hemocyte proliferation [GO:0035207], positive regulation of hemocyte proliferation [GO:0035208]